{
  "gene_symbol": "TYW5",
  "term_id": "GO:0031591",
  "gene_name": "tRNA wybutosine-synthesizing protein 5",
  "term_label": "wybutosine biosynthetic process",
  "gene": "UniProtKB:A2RUC4"
}